{
  "gene_name": "Death domain-containing protein CRADD",
  "gene_symbol": "CRADD",
  "term_label": "positive regulation of apoptotic signaling pathway",
  "term_id": "GO:2001235",
  "gene": "UniProtKB:P78560"
}